{
  "term_id": "UNKNOWN:0001",
  "gene_name": "Protein EOLA2",
  "gene_symbol": "EOLA2",
  "gene": "UniProtKB:Q96DE9",
  "term_label": "Unknown molecular function"
}